{
  "gene_name": "Bifunctional arginine demethylase and lysyl-hydroxylase JMJD6",
  "term_id": "GO:0005737",
  "gene_symbol": "JMJD6",
  "term_label": "cytoplasm",
  "gene": "UniProtKB:Q6NYC1"
}